{
  "gene_name": "Olfactory receptor 1I1",
  "gene_symbol": "OR1I1",
  "term_label": "plasma membrane",
  "term_id": "GO:0005886",
  "gene": "UniProtKB:O60431"
}